{
  "term_label": "DNA-binding transcription factor activity, RNA polymerase II-specific",
  "gene_symbol": "FOXA1",
  "gene_name": "Hepatocyte nuclear factor 3-alpha",
  "gene": "UniProtKB:P55317",
  "term_id": "GO:0000981"
}